{
  "gene_symbol": "SLFN12",
  "gene_name": "Ribonuclease SLFN12",
  "term_label": "Unknown cellular component",
  "gene": "UniProtKB:Q8IYM2",
  "term_id": "UNKNOWN:0003"
}